rhombomere 7 development [GO:0021573] (biological process) Sources: GOC:cls, GOC:curators, GOC:dgh, GOC:dph, GOC:jid Relationships: is a type of GO:0021546 Definition: The process whose specific outcome is the progression of rhombomere 7 over time, from its formation to the mature structure. Rhombomeres are transverse segments of the developing rhombencephalon. Rhombomeres are lineage restricted, express different genes from one another, and adopt different developmental fates. Rhombomeres are numbered in anterior to posterior order.